MHC class I protein complex binding [GO:0023024] (molecular function) Definition: Binding to a class I major histocompatibility complex. Sources: GOC:mtg_signal, GOC:vw Relationships: is a type of MHC protein complex binding [GO:0023023]